{
  "term_label": "Unknown molecular function",
  "gene_symbol": "VSTM2B",
  "gene": "UniProtKB:A6NLU5",
  "term_id": "UNKNOWN:0001",
  "gene_name": "V-set and transmembrane domain-containing protein 2B"
}